{
  "term_id": "GO:0000978",
  "gene": "UniProtKB:Q8N196",
  "term_label": "RNA polymerase II cis-regulatory region sequence-specific DNA binding",
  "gene_symbol": "SIX5",
  "gene_name": "Homeobox protein SIX5"
}